{
  "gene_symbol": "SPANXN3",
  "gene": "UniProtKB:Q5MJ09",
  "term_id": "UNKNOWN:0001",
  "term_label": "Unknown molecular function",
  "gene_name": "Sperm protein associated with the nucleus on the X chromosome N3"
}